{
  "term_label": "Unknown molecular function",
  "gene_symbol": "BLID",
  "term_id": "UNKNOWN:0001",
  "gene": "UniProtKB:Q8IZY5",
  "gene_name": "BH3-like motif-containing cell death inducer"
}